{
  "gene_symbol": "NXNL2",
  "gene": "UniProtKB:Q5VZ03",
  "term_label": "sensory perception of smell",
  "term_id": "GO:0007608",
  "gene_name": "Nucleoredoxin-like protein 2"
}